{
  "gene": "UniProtKB:Q15223",
  "term_id": "GO:1902414",
  "gene_name": "Nectin-1",
  "gene_symbol": "NECTIN1",
  "term_label": "protein localization to cell junction"
}